{
  "gene_name": "E3 ubiquitin-protein ligase RNF180",
  "term_id": "GO:0032436",
  "term_label": "positive regulation of proteasomal ubiquitin-dependent protein catabolic process",
  "gene_symbol": "RNF180",
  "gene": "UniProtKB:Q86T96"
}